{
  "gene_name": "Cilia- and flagella-associated protein 141",
  "term_id": "UNKNOWN:0001",
  "gene": "UniProtKB:Q5VU69",
  "gene_symbol": "CFAP141",
  "term_label": "Unknown molecular function"
}